regulation of small GTPase mediated signal transduction [GO:0051056] (biological process) Also known as: regulation of small GTPase-mediated signal transduction Definition: Any process that modulates the frequency, rate or extent of small GTPase mediated signal transduction. Sources: GOC:go_curators Relationships: is a type of GO:1902531; regulates small GTPase-mediated signal transduction [GO:0007264] Subtypes: regulation of septation initiation signaling [GO:0031029], regulation of ARF protein signal transduction [GO:0032012], regulation of Rab protein signal transduction [GO:0032483], GO:0032485, GO:0032487, GO:0035020, regulation of Rho protein signal transduction [GO:0035023], symbiont-mediated perturbation of host small GTPase-mediated signal transduction [GO:0044082], regulation of Ras protein signal transduction [GO:0046578], positive regulation of small GTPase mediated signal transduction [GO:0051057], negative regulation of small GTPase mediated signal transduction [GO:0051058]